{
  "gene": "UniProtKB:Q9Y666",
  "gene_symbol": "SLC12A7",
  "gene_name": "Solute carrier family 12 member 7",
  "term_id": "GO:0006884",
  "term_label": "cell volume homeostasis"
}